{
  "gene": "UniProtKB:Q15172",
  "term_id": "UNKNOWN:0002",
  "gene_name": "Serine_threonine-protein phosphatase 2A 56 kDa regulatory subunit alpha isoform",
  "term_label": "Unknown biological process",
  "gene_symbol": "PPP2R5A"
}